{
  "term_id": "GO:0050728",
  "gene_symbol": "NR1H3",
  "gene": "UniProtKB:Q13133",
  "gene_name": "Oxysterols receptor LXR-alpha",
  "term_label": "negative regulation of inflammatory response"
}